{
  "term_id": "UNKNOWN:0003",
  "gene": "UniProtKB:Q9UKL6",
  "gene_symbol": "PCTP",
  "term_label": "Unknown cellular component",
  "gene_name": "Phosphatidylcholine transfer protein"
}